{
  "gene": "UniProtKB:P78509",
  "term_label": "neuron projection",
  "gene_symbol": "RELN",
  "term_id": "GO:0043005",
  "gene_name": "Reelin"
}